{
  "gene": "UniProtKB:K7EIQ3",
  "term_id": "UNKNOWN:0002",
  "gene_symbol": "ZNF561-AS1",
  "gene_name": "Uncharacterized protein ZNF561-AS1",
  "term_label": "Unknown biological process"
}